{
  "gene": "UniProtKB:Q15796",
  "term_id": "GO:0070411",
  "term_label": "I-SMAD binding",
  "gene_symbol": "SMAD2",
  "gene_name": "Mothers against decapentaplegic homolog 2"
}